{
  "term_label": "dehydrodolichyl diphosphate synthase complex",
  "gene_name": "Dehydrodolichyl diphosphate synthase complex subunit DHDDS",
  "gene": "UniProtKB:Q86SQ9",
  "term_id": "GO:1904423",
  "gene_symbol": "DHDDS"
}